{
  "term_label": "Wnt-protein binding",
  "gene_symbol": "WLS",
  "gene": "UniProtKB:Q5T9L3",
  "term_id": "GO:0017147",
  "gene_name": "Protein wntless homolog"
}